{
  "gene_name": "T cell receptor beta variable 11-3",
  "gene": "UniProtKB:A0A5A6",
  "term_id": "GO:0007166",
  "term_label": "cell surface receptor signaling pathway",
  "gene_symbol": "TRBV11-3"
}